{
  "gene_name": "E3 ubiquitin-protein ligase RNF25",
  "term_label": "ubiquitin protein ligase activity",
  "gene": "UniProtKB:Q96BH1",
  "gene_symbol": "RNF25",
  "term_id": "GO:0061630"
}